lysosomal glycocalyx [GO:0090123] (cellular component) Relationships: is a type of glycocalyx [GO:0030112]; is part of GO:0005764 Definition: The polysaccharide-based coating on the inner side of a lysosomal membrane. It may be involved in protecting the membrane from digestion by lysosomal enzymes. References: PMID:10521503, PMID:22809326, PMID:29367433 Sources: GOC:ascb_2009, GOC:dph, GOC:krc, GOC:tb